phototaxis [GO:0042331] (biological process) Subtypes: positive phototaxis [GO:0046956], negative phototaxis [GO:0046957] Definition: The directed movement of a motile cell or organism in response to light. Relationships: is a type of response to light stimulus [GO:0009416]; is a type of GO:0009453 Also known as: phototactic behavior, phototactic behaviour, taxis in response to light Sources: GOC:jl, ISBN:0192800981